testosterone dehydrogenase (NADP+) activity [GO:0047045] (molecular function) Also known as: 17-ketoreductase activity, 17beta-hydroxysteroid:NADP+ 17-oxidoreductase activity, NADP-dependent testosterone-17beta-oxidoreductase activity, testosterone 17-beta-dehydrogenase (NADP+) activity, testosterone 17beta-dehydrogenase (NADP+) Definition: Catalysis of the reaction: NADP+ + testosterone = NADPH + H+ + androst-4-ene-3,17-dione. Sources: EC:1.1.1.64 Relationships: is a type of 17-beta-hydroxysteroid dehydrogenase (NADP+) activity [GO:0072582]